{
  "term_label": "Unknown biological process",
  "gene_symbol": "AKR1B15",
  "term_id": "UNKNOWN:0002",
  "gene": "UniProtKB:C9JRZ8",
  "gene_name": "Aldo-keto reductase family 1 member B15"
}